{
  "gene_name": "Granule associated Rac and RHOG effector protein 1",
  "gene": "UniProtKB:O15063",
  "gene_symbol": "GARRE1",
  "term_id": "GO:1905762",
  "term_label": "CCR4-NOT complex binding"
}